{
  "term_id": "GO:0051932",
  "gene_symbol": "GABRR2",
  "gene": "UniProtKB:P28476",
  "term_label": "synaptic transmission, GABAergic",
  "gene_name": "Gamma-aminobutyric acid receptor subunit rho-2"
}